{
  "gene": "UniProtKB:Q9H6U8",
  "term_label": "protein N-linked glycosylation",
  "gene_symbol": "ALG9",
  "term_id": "GO:0006487",
  "gene_name": "Alpha-1,2-mannosyltransferase ALG9"
}